regulation of glutathione biosynthetic process [GO:1903786] (biological process) Definition: Any process that modulates the frequency, rate or extent of glutathione biosynthetic process. Also known as: regulation of glutathione anabolism, regulation of glutathione biosynthesis, regulation of glutathione formation, regulation of glutathione synthesis Relationships: is a type of regulation of biosynthetic process [GO:0009889]; is a type of GO:0034248; is a type of regulation of sulfur metabolic process [GO:0042762]; regulates GO:0006750 Subtypes: negative regulation of glutathione biosynthetic process [GO:1903787], positive regulation of glutathione biosynthetic process [GO:1903788] Sources: GOC:PARL, GOC:TermGenie, GOC:bf, GO_REF:0000058